negative regulation of cell motility [GO:2000146] (biological process) Sources: GOC:mah Also known as: negative regulation of cell locomotion, negative regulation of movement of a cell, negative regulation of cell movement Relationships: is_a GO:0040013; is a type of negative regulation of cellular process [GO:0048523]; is a type of regulation of cell motility [GO:2000145]; negatively regulates GO:0048870 Definition: Any process that stops, prevents, or reduces the frequency, rate or extent of cell motility. Subtypes: negative regulation of cell migration [GO:0030336], negative regulation of cilium-dependent cell motility [GO:1902020], GO:1902201, negative regulation of amoeboid sperm motility [GO:1905417]